{
  "term_id": "GO:0006303",
  "gene_symbol": "PAXX",
  "gene_name": "Protein PAXX",
  "gene": "UniProtKB:Q9BUH6",
  "term_label": "double-strand break repair via nonhomologous end joining"
}